{
  "gene": "UniProtKB:Q15149",
  "gene_symbol": "PLEC",
  "term_label": "hemidesmosome assembly",
  "term_id": "GO:0031581",
  "gene_name": "Plectin"
}